membrane microdomain [GO:0098857] (cellular component) Relationships: is_a membrane [GO:0016020] Definition: A membrane region with a lipid composition that is distinct from that of the membrane regions that surround it. Subtypes: membrane raft [GO:0045121], caveola neck [GO:0099400], caveola bulb [GO:0099401] References: PMID:20044567, PMID:26253820